{
  "term_label": "Unknown molecular function",
  "gene": "UniProtKB:Q9P1C3",
  "term_id": "UNKNOWN:0001",
  "gene_name": "Putative uncharacterized protein PRO2829",
  "gene_symbol": "PRO2829"
}